catalase complex [GO:0062151] (cellular component) Definition: A protein-containing complex that is capable of catalase activity. Relationships: is_a oxidoreductase complex [GO:1990204] References: PMID:10656833 Sources: GOC:bhm